host cell nucleoplasm [GO:0044095] (cellular component) Relationships: is a type of host cell nuclear part [GO:0044094] Definition: That part of a host cell's nuclear content other than the chromosomes or the nucleolus. The host is the larger of the organisms involved in a symbiotic interaction. Sources: GOC:ecd